{
  "gene_symbol": "SBNO2",
  "gene_name": "Protein strawberry notch homolog 2",
  "term_label": "nucleus",
  "gene": "UniProtKB:Q9Y2G9",
  "term_id": "GO:0005634"
}